{
  "gene_symbol": "ATF2",
  "term_id": "GO:0035497",
  "term_label": "cAMP response element binding",
  "gene_name": "Cyclic AMP-dependent transcription factor ATF-2",
  "gene": "UniProtKB:P15336"
}